{
  "gene_name": "HLA class II histocompatibility antigen, DQ beta 1 chain",
  "term_label": "antigen processing and presentation of exogenous peptide antigen via MHC class II",
  "gene": "UniProtKB:P01920",
  "gene_symbol": "HLA-DQB1",
  "term_id": "GO:0019886"
}